{
  "term_label": "DNA-binding transcription factor activity, RNA polymerase II-specific",
  "gene_symbol": "WT1",
  "gene": "UniProtKB:P19544",
  "term_id": "GO:0000981",
  "gene_name": "Wilms tumor protein"
}